{
  "gene": "UniProtKB:Q7Z5A9",
  "gene_symbol": "TAFA1",
  "term_id": "GO:0048018",
  "term_label": "receptor ligand activity",
  "gene_name": "Chemokine-like protein TAFA-1"
}